{
  "gene_name": "Olfactory receptor 8J2",
  "term_id": "UNKNOWN:0002",
  "gene": "UniProtKB:Q8NGG1",
  "term_label": "Unknown biological process",
  "gene_symbol": "OR8J2"
}